{
  "gene_name": "Keratin, type I cytoskeletal 40",
  "term_label": "epithelial cell differentiation",
  "term_id": "GO:0030855",
  "gene": "UniProtKB:Q6A162",
  "gene_symbol": "KRT40"
}